{
  "gene_symbol": "GTF2F2",
  "gene_name": "General transcription factor IIF subunit 2",
  "term_id": "UNKNOWN:0001",
  "gene": "UniProtKB:P13984",
  "term_label": "Unknown molecular function"
}